nicotinamide nucleotide biosynthetic process from niacinamide [GO:0019360] (biological process) Sources: GOC:go_curators Also known as: nicotinamide nucleotide anabolism from niacinamide, nicotinamide nucleotide formation from niacinamide, nicotinamide nucleotide synthesis from niacinamide Relationships: is a type of GO:0006769; is a type of nicotinamide nucleotide biosynthetic process [GO:0019359] Definition: The chemical reactions and pathways resulting in the formation of nicotinamide nucleotide from other compounds, including niacinamide.